{
  "term_label": "ceramide catabolic process",
  "gene_name": "Alkaline ceramidase 2",
  "gene": "UniProtKB:Q5QJU3",
  "gene_symbol": "ACER2",
  "term_id": "GO:0046514"
}